{
  "gene_symbol": "VRTN",
  "term_id": "UNKNOWN:0001",
  "term_label": "Unknown molecular function",
  "gene_name": "Vertnin",
  "gene": "UniProtKB:Q9H8Y1"
}